positive regulation of transcytosis [GO:1904300] (biological process) Definition: Any process that activates or increases the frequency, rate or extent of transcytosis. Also known as: up regulation of transcytosis, up-regulation of transcytosis, upregulation of transcytosis, activation of transcytosis Relationships: is a type of positive regulation of cellular process [GO:0048522]; is a type of positive regulation of transport [GO:0051050]; is_a GO:0051240; is a type of regulation of transcytosis [GO:1904298]; positively regulates transcytosis [GO:0045056] References: PMID:9664076 Sources: GOC:TermGenie, GO_REF:0000058